regulation of reverse cholesterol transport [GO:1903062] (biological process) Definition: Any process that modulates the frequency, rate or extent of reverse cholesterol transport. References: PMID:23931754 Sources: GOC:BHF, GOC:TermGenie, GOC:rl, GO_REF:0000058 Subtypes: GO:1903063, GO:1903064 Relationships: is a type of regulation of cholesterol transport [GO:0032374]; regulates reverse cholesterol transport [GO:0043691]